Gly-tRNA(Ala) deacylase activity [GO:0106026] (molecular function) References: PMID:28362257 Sources: RHEA:53744 Definition: Catalysis of the reaction: glycyl-tRNA(Ala) + H2O = tRNA(Ala) + glycine + H+. Relationships: is a type of aminoacyl-tRNA deacylase activity [GO:0002161]